{
  "term_label": "cell surface receptor signaling pathway",
  "term_id": "GO:0007166",
  "gene_name": "T cell receptor beta variable 20-1",
  "gene_symbol": "TRBV20-1",
  "gene": "UniProtKB:A0A075B6N2"
}